{
  "term_label": "glutathione metabolic process",
  "gene": "UniProtKB:O15217",
  "gene_symbol": "GSTA4",
  "term_id": "GO:0006749",
  "gene_name": "Glutathione S-transferase A4"
}